{
  "term_id": "GO:0061025",
  "gene_name": "E3 ubiquitin-protein ligase HUWE1",
  "gene_symbol": "HUWE1",
  "gene": "UniProtKB:Q7Z6Z7",
  "term_label": "membrane fusion"
}